{
  "gene_symbol": "RCSD1",
  "gene_name": "CapZ-interacting protein",
  "gene": "UniProtKB:Q6JBY9",
  "term_id": "GO:0071203",
  "term_label": "WASH complex"
}